{
  "term_id": "GO:0017157",
  "gene": "UniProtKB:Q9ULW5",
  "term_label": "regulation of exocytosis",
  "gene_symbol": "RAB26",
  "gene_name": "Ras-related protein Rab-26"
}